cholangiocyte proliferation [GO:1990705] (biological process) References: PMID:24434010 Relationships: is_a GO:0050673 Definition: The multiplication or reproduction of cholangiocytes, resulting in the expansion of the cholangiocyte population. A cholangiocyte is an epithelial cell that is part of the bile duct. Cholangiocytes contribute to bile secretion via net release of bicarbonate and water. Regulation: regulated by regulation of cholangiocyte proliferation [GO:1904054]; negatively regulated by GO:1904055; positively regulated by positive regulation of cholangiocyte proliferation [GO:1904056] Also known as: hepatoblast proliferation